Sertoli cell differentiation [GO:0060008] (biological process) Definition: The process in which a relatively unspecialized cell acquires specialized structural and/or functional features of a Sertoli cell. A Sertoli cell is a supporting cell projecting inward from the basement membrane of seminiferous tubules. Sources: GOC:dph Relationships: is a type of developmental process involved in reproduction [GO:0003006]; is a type of GO:0030855; is part of male gonad development [GO:0008584]